{
  "term_label": "filamentous actin",
  "gene_symbol": "PDLIM7",
  "term_id": "GO:0031941",
  "gene": "UniProtKB:Q9NR12",
  "gene_name": "PDZ and LIM domain protein 7"
}